{
  "term_id": "GO:0005128",
  "gene_symbol": "EPO",
  "gene_name": "Erythropoietin",
  "term_label": "erythropoietin receptor binding",
  "gene": "UniProtKB:P01588"
}